{
  "term_label": "nucleolus",
  "gene": "UniProtKB:Q14978",
  "gene_symbol": "NOLC1",
  "gene_name": "Nucleolar and coiled-body phosphoprotein 1",
  "term_id": "GO:0005730"
}